{
  "gene_symbol": "MRPS7",
  "gene_name": "Small ribosomal subunit protein uS7m",
  "term_id": "GO:0019843",
  "term_label": "rRNA binding",
  "gene": "UniProtKB:Q9Y2R9"
}